{
  "gene": "UniProtKB:Q92804",
  "gene_name": "TATA-binding protein-associated factor 2N",
  "term_label": "nucleus",
  "gene_symbol": "TAF15",
  "term_id": "GO:0005634"
}